thiamine import across plasma membrane [GO:0140125] (biological process) Relationships: is a type of thiamine transmembrane transport [GO:0071934]; is_a import across plasma membrane [GO:0098739] Sources: GOC:vw Definition: The directed movement of thiamine from outside of a cell, across the plasma membrane and into the cytosol.